{
  "gene_name": "Thymidine kinase 2, mitochondrial",
  "gene": "UniProtKB:O00142",
  "term_label": "Unknown biological process",
  "gene_symbol": "TK2",
  "term_id": "UNKNOWN:0002"
}